{
  "gene": "UniProtKB:Q9H1E1",
  "gene_name": "Ribonuclease 7",
  "term_label": "defense response to Gram-positive bacterium",
  "term_id": "GO:0050830",
  "gene_symbol": "RNASE7"
}